cystic duct development [GO:0035628] (biological process) References: PMID:20614624 Relationships: is a type of common bile duct development [GO:0061009] Definition: The progression of the cystic duct over time, from its formation to the mature structure. The cystic duct runs from the gallbladder to the common bile duct.